{
  "term_id": "GO:0005789",
  "gene_name": "Stearoyl-CoA desaturase 5",
  "gene_symbol": "SCD5",
  "gene": "UniProtKB:Q86SK9",
  "term_label": "endoplasmic reticulum membrane"
}